{
  "term_id": "UNKNOWN:0001",
  "term_label": "Unknown molecular function",
  "gene_name": "Coatomer subunit epsilon",
  "gene_symbol": "COPE",
  "gene": "UniProtKB:O14579"
}